{
  "gene_name": "T-cell surface glycoprotein CD1e, membrane-associated",
  "term_id": "GO:0048006",
  "gene": "UniProtKB:P15812",
  "gene_symbol": "CD1E",
  "term_label": "antigen processing and presentation, endogenous lipid antigen via MHC class Ib"
}